positive regulation of sodium ion export across plasma membrane [GO:1903278] (biological process) Definition: Any process that activates or increases the frequency, rate or extent of sodium ion export across the plasma membrane. References: PMID:17095720 Sources: GOC:BHF, GOC:TermGenie, GOC:rl, GO_REF:0000058 Also known as: positive regulation of sodium ion export from cell, up regulation of sodium ion export from cell, up-regulation of sodium ion export from cell, upregulation of sodium ion export from cell, activation of sodium export, activation of sodium ion export, activation of sodium ion export from cell, positive regulation of sodium export, positive regulation of sodium ion export, up regulation of sodium export, up regulation of sodium ion export, up-regulation of sodium export, up-regulation of sodium ion export, upregulation of sodium export, upregulation of sodium ion export Relationships: is a type of positive regulation of sodium ion transmembrane transport [GO:1902307]; is a type of GO:1903276; positively regulates sodium ion export across plasma membrane [GO:0036376]